tartrate dehydrogenase activity [GO:0009027] (MF) Also known as: mesotartrate dehydrogenase activity, tartrate:NAD+ oxidoreductase activity Relationships: is a type of GO:0016616 Sources: EC:1.1.1.93 Definition: Catalysis of the reaction: tartrate + NAD+ = oxaloglycolate + NADH + H+.